{
  "term_id": "GO:0005634",
  "gene_symbol": "USP17L17",
  "gene": "UniProtKB:D6RBQ6",
  "term_label": "nucleus",
  "gene_name": "Ubiquitin carboxyl-terminal hydrolase 17-like protein 17"
}